negative regulation of embryonic camera-type eye development [GO:1902864] (biological process) References: PMID:16872597 Sources: GOC:TermGenie, GOC:mr, GO_REF:0000058 Relationships: is a type of negative regulation of developmental process [GO:0051093]; is a type of regulation of embryonic camera-type eye development [GO:1902863]; negatively regulates embryonic camera-type eye development [GO:0031076] Definition: Any process that stops, prevents or reduces the frequency, rate or extent of embryonic camera-type eye development. Also known as: down regulation of embryonic camera-type eye development, down regulation of embryonic eye development, down-regulation of embryonic camera-type eye development, down-regulation of embryonic eye development, downregulation of embryonic camera-type eye development, downregulation of embryonic eye development, negative regulation of embryonic eye development, inhibition of embryonic camera-type eye development, inhibition of embryonic eye development